{
  "term_label": "RNA binding",
  "term_id": "GO:0003723",
  "gene": "UniProtKB:Q6PKG0",
  "gene_name": "La-related protein 1",
  "gene_symbol": "LARP1"
}